fungal-type cell wall organization or biogenesis [GO:0071852] (biological process) Subtypes: fungal-type cell wall biogenesis [GO:0009272], fungal-type cell wall organization [GO:0031505] Sources: GOC:mah Definition: A process that results in the biosynthesis of constituent macromolecules, assembly, arrangement of constituent parts, or disassembly of a fungal-type cell wall. Relationships: is a type of cell wall organization or biogenesis [GO:0071554] Also known as: fungal-type cell wall organisation or biogenesis, fungal-type cell wall organization and biogenesis